{
  "term_id": "GO:0005254",
  "gene_name": "Gamma-aminobutyric acid receptor subunit alpha-5",
  "term_label": "chloride channel activity",
  "gene": "UniProtKB:P31644",
  "gene_symbol": "GABRA5"
}